regulation of myofibril number [GO:0014882] (biological process) Also known as: change of myofibril number Definition: Any process that modulates the number of myofibrils. A myofibril is the contractile element of skeletal and cardiac muscle. It is a long, highly organized bundle of actin, myosin, and other proteins that contracts by a sliding filament mechanism. Relationships: is a type of regulation of muscle hyperplasia [GO:0014738]; is a type of regulation of biological quality [GO:0065008] Sources: GOC:dph, GOC:ef, GOC:mtg_muscle, GOC:tb